{
  "term_label": "Unknown cellular component",
  "term_id": "UNKNOWN:0003",
  "gene": "UniProtKB:Q6IC83",
  "gene_name": "Uncharacterized protein C22orf42",
  "gene_symbol": "C22orf42"
}